negative regulation of bone resorption [GO:0045779] (BP) Sources: GOC:go_curators Definition: Any process that stops, prevents, or reduces the frequency, rate or extent of bone resorption. Also known as: down regulation of bone resorption, down-regulation of bone resorption, downregulation of bone resorption, inhibition of bone resorption Relationships: is a type of GO:0045124; is_a GO:0046851; negatively regulates bone resorption [GO:0045453]